{
  "gene_symbol": "FIGNL1",
  "gene": "UniProtKB:Q6PIW4",
  "term_label": "microtubule severing ATPase activity",
  "term_id": "GO:0008568",
  "gene_name": "Fidgetin-like protein 1"
}